{
  "gene": "UniProtKB:Q9UHP9",
  "term_id": "UNKNOWN:0001",
  "gene_name": "Small muscular protein",
  "gene_symbol": "SMPX",
  "term_label": "Unknown molecular function"
}